{
  "term_label": "regulation of autophagy",
  "term_id": "GO:0010506",
  "gene_name": "DNA damage-regulated autophagy modulator protein 1",
  "gene_symbol": "DRAM1",
  "gene": "UniProtKB:Q8N682"
}